slow axonal transport [GO:1990832] (biological process) Definition: The directed slow movement of non-membranous molecules in nerve cell axons. It is comprised of a Slow Component a (SCa) and a Slow Component b (SCb) which differ in transport rates and protein composition. References: PMID:6378920 Relationships: is_a axo-dendritic transport [GO:0008088]